{
  "gene": "UniProtKB:P19022",
  "term_id": "GO:0030027",
  "gene_symbol": "CDH2",
  "term_label": "lamellipodium",
  "gene_name": "Cadherin-2"
}